{
  "term_label": "detection of chemical stimulus involved in sensory perception of smell",
  "gene_name": "Olfactory receptor 13D1",
  "term_id": "GO:0050911",
  "gene_symbol": "OR13D1",
  "gene": "UniProtKB:Q8NGV5"
}